dorsal aorta development [GO:0035907] (biological process) Definition: The progression of the dorsal aorta over time, from its initial formation to the mature structure. The dorsal aorta is a blood vessel in a single-pass circulatory system that carries oxygenated blood from the gills to the rest of the body. In a single-pass circulatory system blood passes once through the heart to supply the body once. Sources: GOC:bf, GOC:dgh, UBERON:0005805, Wikipedia:Aorta, ZFA:0000014 Relationships: is a type of aorta development [GO:0035904]